negative regulation of protein serine/threonine kinase activity [GO:0071901] (biological process) Sources: GOC:BHF, GOC:mah Relationships: is a type of GO:0006469; is_a GO:0071900; negatively regulates protein serine/threonine kinase activity [GO:0004674] Subtypes: GO:0043407, negative regulation of cyclin-dependent protein serine/threonine kinase activity [GO:0045736], negative regulation of Rho-dependent protein serine/threonine kinase activity [GO:2000299], negative regulation of cAMP-dependent protein kinase activity [GO:2000480] Definition: Any process that decreases the rate, frequency, or extent of protein serine/threonine kinase activity.